{
  "gene": "UniProtKB:Q8NCS7",
  "gene_symbol": "SLC44A5",
  "term_id": "GO:0016020",
  "term_label": "membrane",
  "gene_name": "Choline transporter-like protein 5"
}